omega-hydroxylase P450 pathway [GO:0097267] (BP) Definition: The chemical reactions and pathways by which arachidonic acid is converted to other compounds initially by omega-hydroxylation. References: PMID:10681399 Sources: GOC:mw Relationships: is_a GO:0019369 Also known as: P450 omega-hydroxylase pathway